{
  "gene_symbol": "KDM3A",
  "gene": "UniProtKB:Q9Y4C1",
  "term_id": "GO:0003712",
  "gene_name": "Lysine-specific demethylase 3A",
  "term_label": "transcription coregulator activity"
}